{
  "term_label": "intracellular signal transduction",
  "gene_name": "T-cell leukemia_lymphoma protein 1B",
  "gene": "UniProtKB:O95988",
  "gene_symbol": "TCL1B",
  "term_id": "GO:0035556"
}